{
  "gene": "UniProtKB:P20963",
  "gene_name": "T-cell surface glycoprotein CD3 zeta chain",
  "gene_symbol": "CD247",
  "term_label": "T cell receptor signaling pathway",
  "term_id": "GO:0050852"
}